intraciliary anterograde transport [GO:0035720] (biological process) Also known as: intraflagellar anterograde transport Definition: The directed movement of large protein complexes along microtubules from the cell body toward the tip of a cilium (also called flagellum), mediated by motor proteins. Relationships: is a type of intraciliary transport [GO:0042073] Note: Note that we deem cilium and microtubule-based flagellum to be equivalent. Regulation: regulated by regulation of intraciliary anterograde transport [GO:1905796]; negatively regulated by negative regulation of intraciliary anterograde transport [GO:1905797]; positively regulated by positive regulation of intraciliary anterograde transport [GO:1905798] References: PMID:17895364 Sources: GOC:BHF, GOC:cilia